{
  "gene_symbol": "RAC3",
  "term_label": "actin filament organization",
  "gene_name": "Ras-related C3 botulinum toxin substrate 3",
  "gene": "UniProtKB:P60763",
  "term_id": "GO:0007015"
}